{
  "gene_symbol": "OR2A7",
  "term_id": "GO:0005549",
  "gene_name": "Olfactory receptor 2A7",
  "term_label": "odorant binding",
  "gene": "UniProtKB:Q96R45"
}